{
  "term_id": "GO:0005085",
  "gene": "UniProtKB:Q7LDG7",
  "gene_name": "RAS guanyl-releasing protein 2",
  "term_label": "guanyl-nucleotide exchange factor activity",
  "gene_symbol": "RASGRP2"
}